symbiont-mediated evasion of recognition by host complement [GO:0141178] (biological process) Relationships: is a type of symbiont-mediated evasion of recognition by host innate immune effector [GO:0141177] Definition: A process by which a symbiont avoids the effects of recognition by host  complement by altering molecules on the symbiont surface. The host is defined as the larger of the organisms involved in a symbiotic interaction. Also known as: symbiont-mediated evasion of host complement References: PMID:22825444, PMID:25537831, PMID:34887398